ATPase activator activity [GO:0001671] (molecular function) Relationships: is a type of ATPase regulator activity [GO:0060590]; is a type of GO:0140677; positively regulates ATP-dependent activity [GO:0140657] Sources: GOC:ajp Also known as: ATPase stimulator activity Subtypes: DNA topoisomerase type II (double strand cut, ATP-hydrolyzing) activator activity [GO:0072587] Definition: Binds to and increases the activity of an ATP hydrolysis activity.